{
  "gene_symbol": "SMIM41",
  "gene": "UniProtKB:A0A2R8YCJ5",
  "term_label": "Unknown biological process",
  "term_id": "UNKNOWN:0002",
  "gene_name": "Small integral membrane protein 41"
}